{
  "gene": "UniProtKB:P61244",
  "gene_symbol": "MAX",
  "term_id": "GO:0045944",
  "gene_name": "Protein max",
  "term_label": "positive regulation of transcription by RNA polymerase II"
}